{
  "gene_name": "Fibronectin type III and SPRY domain-containing protein 1",
  "gene_symbol": "FSD1",
  "term_label": "regulation of mitotic spindle organization",
  "term_id": "GO:0060236",
  "gene": "UniProtKB:Q9BTV5"
}